positive regulation of gamma-delta T cell activation [GO:0046645] (biological process) Definition: Any process that activates or increases the frequency, rate or extent of gamma-delta T cell activation. Subtypes: positive regulation of gamma-delta T cell differentiation [GO:0045588], positive regulation of gamma-delta T cell proliferation [GO:0046648], positive regulation of gamma-delta T cell activation involved in immune response [GO:2001193] Relationships: is_a regulation of gamma-delta T cell activation [GO:0046643]; is a type of positive regulation of T cell activation [GO:0050870]; positively regulates GO:0046629 Sources: GOC:ai Also known as: positive regulation of gamma-delta T lymphocyte activation, positive regulation of gamma-delta T-cell activation, positive regulation of gamma-delta T-lymphocyte activation, up regulation of gamma-delta T cell activation, up-regulation of gamma-delta T cell activation, upregulation of gamma-delta T cell activation, activation of gamma-delta T cell activation, stimulation of gamma-delta T cell activation